{
  "term_id": "GO:0000981",
  "gene_name": "Zinc finger protein 302",
  "gene": "UniProtKB:Q9NR11",
  "term_label": "DNA-binding transcription factor activity, RNA polymerase II-specific",
  "gene_symbol": "ZNF302"
}